{
  "term_label": "cell motility",
  "gene_name": "POTE ankyrin domain family member F",
  "term_id": "GO:0048870",
  "gene": "UniProtKB:A5A3E0",
  "gene_symbol": "POTEF"
}